{
  "term_label": "endoplasmic reticulum-plasma membrane tethering",
  "gene_name": "Vesicle-associated membrane protein-associated protein B_C",
  "gene_symbol": "VAPB",
  "gene": "UniProtKB:O95292",
  "term_id": "GO:0061817"
}